{
  "gene": "UniProtKB:Q8NFR7",
  "term_label": "Unknown cellular component",
  "gene_symbol": "CCDC148",
  "gene_name": "Coiled-coil domain-containing protein 148",
  "term_id": "UNKNOWN:0003"
}